{
  "gene_symbol": "AMPD3",
  "term_label": "AMP metabolic process",
  "term_id": "GO:0046033",
  "gene": "UniProtKB:Q01432",
  "gene_name": "AMP deaminase 3"
}